NAD+-protein-glutamate ADP-ribosyltransferase activity [GO:0140807] (MF) References: PMID:19764761, PMID:25043379 Sources: RHEA:58224 Relationships: is a type of NAD+-protein mono-ADP-ribosyltransferase activity [GO:1990404] Subtypes: NAD+-histone H2BE35 glutamate ADP-ribosyltransferase activity [GO:0140822], GO:0140844 Definition: Catalysis of the reaction: L-glutamyl-[protein] + NAD+ = 5-O-(ADP-D-ribosyl)-L-glutamyl-[protein] + nicotinamide.